response to copper ion starvation [GO:0120126] (BP) Relationships: is a type of response to metal ion starvation [GO:0180055] Subtypes: cellular response to copper ion starvation [GO:0035874] References: PMID:24024382 Sources: GOC:sl Definition: Any process that results in a change in state or activity of a cell or an organism (in terms of movement, secretion, enzyme production, gene expression, etc.) as a result of a starvation stimulus, deprivation of copper ion.